{
  "gene_symbol": "COMT",
  "gene": "UniProtKB:P21964",
  "term_label": "membrane",
  "gene_name": "Catechol O-methyltransferase",
  "term_id": "GO:0016020"
}